{
  "term_id": "GO:0080025",
  "gene": "UniProtKB:Q9Y484",
  "term_label": "phosphatidylinositol-3,5-bisphosphate binding",
  "gene_symbol": "WDR45",
  "gene_name": "WD repeat domain phosphoinositide-interacting protein 4"
}